{
  "term_label": "arachidonate-CoA ligase activity",
  "gene_name": "Long-chain-fatty-acid--CoA ligase 1",
  "gene": "UniProtKB:P33121",
  "gene_symbol": "ACSL1",
  "term_id": "GO:0047676"
}